{
  "gene_name": "Transmembrane protein 192",
  "gene": "UniProtKB:Q8IY95",
  "term_id": "UNKNOWN:0001",
  "gene_symbol": "TMEM192",
  "term_label": "Unknown molecular function"
}